{
  "gene": "UniProtKB:Q8IWU4",
  "gene_name": "Proton-coupled zinc antiporter SLC30A8",
  "term_label": "response to glucose",
  "gene_symbol": "SLC30A8",
  "term_id": "GO:0009749"
}